{
  "term_label": "Unknown molecular function",
  "term_id": "UNKNOWN:0001",
  "gene_symbol": "MS4A7",
  "gene": "UniProtKB:Q9GZW8",
  "gene_name": "Membrane-spanning 4-domains subfamily A member 7"
}